{
  "gene_symbol": "KCNAB2",
  "term_id": "GO:1901379",
  "term_label": "regulation of potassium ion transmembrane transport",
  "gene_name": "Voltage-gated potassium channel subunit beta-2",
  "gene": "UniProtKB:Q13303"
}